{
  "term_label": "protein phosphatase 1 binding",
  "gene_symbol": "PPP1R3B",
  "gene": "UniProtKB:Q86XI6",
  "gene_name": "Protein phosphatase 1 regulatory subunit 3B",
  "term_id": "GO:0008157"
}